regulation of platelet-derived growth factor receptor-alpha signaling pathway [GO:2000583] (biological process) Sources: GOC:obol Subtypes: negative regulation of platelet-derived growth factor receptor-alpha signaling pathway [GO:2000584], positive regulation of platelet-derived growth factor receptor-alpha signaling pathway [GO:2000585] Also known as: regulation of PDGF receptor-alpha signaling pathway, regulation of alphaPDGF receptor signaling pathway, regulation of platelet-derived growth factor receptor-alpha signalling pathway, regulation of PDGFR-alpha signaling pathway Definition: Any process that modulates the frequency, rate or extent of platelet-derived growth factor receptor-alpha signaling pathway. Relationships: is a type of regulation of platelet-derived growth factor receptor signaling pathway [GO:0010640]; regulates platelet-derived growth factor receptor-alpha signaling pathway [GO:0035790]